{
  "gene_symbol": "NPTN",
  "term_id": "GO:0098632",
  "term_label": "cell-cell adhesion mediator activity",
  "gene_name": "Neuroplastin",
  "gene": "UniProtKB:Q9Y639"
}